{
  "term_id": "GO:0003743",
  "gene_name": "Eukaryotic translation initiation factor 3 subunit D",
  "gene": "UniProtKB:O15371",
  "term_label": "translation initiation factor activity",
  "gene_symbol": "EIF3D"
}